{
  "term_id": "GO:0008284",
  "term_label": "positive regulation of cell population proliferation",
  "gene_symbol": "NRAS",
  "gene_name": "GTPase NRas",
  "gene": "UniProtKB:P01111"
}